{
  "term_label": "cytoplasm",
  "gene_name": "Ropporin-1A",
  "gene_symbol": "ROPN1",
  "gene": "UniProtKB:Q9HAT0",
  "term_id": "GO:0005737"
}